negative regulation of DNA-templated DNA replication [GO:2000104] (BP) Also known as: negative regulation of DNA-dependent DNA replication Relationships: is a type of GO:0008156; is a type of GO:0090329; negatively regulates DNA-templated DNA replication [GO:0006261] Definition: Any process that stops, prevents, or reduces the frequency, rate or extent of DNA-dependent DNA replication. Subtypes: GO:0032297, negative regulation of DNA endoreduplication [GO:0032876], replication fork arrest [GO:0043111], negative regulation of mitochondrial DNA replication [GO:0090298], GO:0110027, negative regulation of nuclear cell cycle DNA replication [GO:1902576] Sources: GOC:mah